{
  "gene_symbol": "AXL",
  "term_label": "cell migration",
  "term_id": "GO:0016477",
  "gene_name": "Tyrosine-protein kinase receptor UFO",
  "gene": "UniProtKB:P30530"
}